{
  "term_id": "UNKNOWN:0002",
  "term_label": "Unknown biological process",
  "gene_name": "Sodium-dependent phosphate transport protein 3",
  "gene_symbol": "SLC17A2",
  "gene": "UniProtKB:O00624"
}